{
  "gene_symbol": "ALDH16A1",
  "term_id": "UNKNOWN:0003",
  "gene_name": "Aldehyde dehydrogenase family 16 member A1",
  "gene": "UniProtKB:Q8IZ83",
  "term_label": "Unknown cellular component"
}